{
  "gene": "UniProtKB:Q86VH2",
  "gene_name": "Kinesin-like protein KIF27",
  "term_id": "GO:0007018",
  "gene_symbol": "KIF27",
  "term_label": "microtubule-based movement"
}